virion attachment to host cell [GO:0019062] (biological process) Definition: The process by which a virion protein binds to molecules on the host cellular surface or host cell surface projection. Also known as: viral absorption, virion attachment to host cell surface receptor, viral attachment to host cell Sources: GOC:bf, GOC:jl, UniProtKB-KW:KW-1161, VZ:956 Relationships: is a type of GO:0044650; is part of viral life cycle [GO:0019058]; BFO_0000051 virion binding [GO:0046790]; has part host cell surface binding [GO:0046812] Subtypes: lipopolysaccharide-mediated virion attachment to host cell [GO:0039638], virion attachment to host cell pilus [GO:0039666], GO:0046813, GO:0046814, virion attachment to host cell flagellum [GO:0098931]